{
  "gene_name": "Unconventional myosin-If",
  "term_id": "GO:0007015",
  "gene_symbol": "MYO1F",
  "term_label": "actin filament organization",
  "gene": "UniProtKB:O00160"
}